catalytic activity, acting on a glycoprotein [GO:0140103] (molecular function) Sources: GOC:molecular_function_refactoring, GOC:pdt Relationships: is_a GO:0140096 Subtypes: alpha-1,3-mannosylglycoprotein 2-beta-N-acetylglucosaminyltransferase activity [GO:0003827], beta-1,3-galactosyl-O-glycosyl-glycoprotein beta-1,6-N-acetylglucosaminyltransferase activity [GO:0003829], beta-1,4-mannosylglycoprotein 4-beta-N-acetylglucosaminyltransferase activity [GO:0003830], glycoprotein-fucosylgalactoside alpha-N-acetylgalactosaminyltransferase activity [GO:0004380], glycoprotein 6-alpha-L-fucosyltransferase activity [GO:0008424], alpha-1,3-mannosylglycoprotein 4-beta-N-acetylglucosaminyltransferase activity [GO:0008454], alpha-1,6-mannosylglycoprotein 2-beta-N-acetylglucosaminyltransferase activity [GO:0008455], glycoprotein-N-acetylgalactosamine 3-beta-galactosyltransferase activity [GO:0016263], glycoprotein 3-alpha-L-fucosyltransferase activity [GO:0018392], GO:0030144, endo-alpha-N-acetylgalactosaminidase activity [GO:0033926], GO:0046525, GO:0047220, beta-1,3-galactosyl-O-glycosyl-glycoprotein beta-1,3-N-acetylglucosaminyltransferase activity [GO:0047223], GO:0047224, GO:0047225, alpha-1,6-mannosylglycoprotein 4-beta-N-acetylglucosaminyltransferase activity [GO:0047253], glucose-1-phospho-D-mannosylglycoprotein phosphodiesterase activity [GO:0047399], GO:0047965 Definition: Catalysis of a biochemical reaction in which one of the substrates is a glycoprotein.